{
  "term_label": "SUMO activating enzyme complex",
  "gene": "UniProtKB:Q9UBT2",
  "term_id": "GO:0031510",
  "gene_symbol": "UBA2",
  "gene_name": "SUMO-activating enzyme subunit 2"
}